{
  "gene": "UniProtKB:Q8IV76",
  "term_label": "CLOCK-BMAL transcription complex",
  "gene_symbol": "PASD1",
  "gene_name": "Circadian clock protein PASD1",
  "term_id": "GO:1990513"
}